{
  "gene": "UniProtKB:Q8N8L6",
  "term_id": "UNKNOWN:0002",
  "gene_name": "ADP-ribosylation factor-like protein 10",
  "term_label": "Unknown biological process",
  "gene_symbol": "ARL10"
}